{
  "gene_name": "Annexin A5",
  "term_label": "calcium-dependent phospholipid binding",
  "gene_symbol": "ANXA5",
  "term_id": "GO:0005544",
  "gene": "UniProtKB:P08758"
}